{
  "term_label": "nucleus",
  "gene_name": "Insulinoma-associated protein 1",
  "gene": "UniProtKB:Q01101",
  "gene_symbol": "INSM1",
  "term_id": "GO:0005634"
}